2-hydroxyquinoline 5,6-dioxygenase activity [GO:0018629] (molecular function) Sources: EC:1.14.12.16 Also known as: 2-oxo-1,2-dihydroquinoline 5,6-dioxygenase activity, quinolin-2(1H)-one 5,6-dioxygenase activity, quinolin-2-ol 5,6-dioxygenase activity, quinolin-2-ol,NADH:oxygen oxidoreductase (5,6-hydroxylating) Relationships: is a type of oxidoreductase activity, acting on paired donors, with incorporation or reduction of molecular oxygen, NAD(P)H as one donor, and incorporation of two atoms of oxygen into one donor [GO:0016708] Definition: Catalysis of the reaction: quinolin-2-ol + NADH + H+ + O2 = 2,5,6-trihydroxy-5,6-dihydroquinoline + NAD+.